18S rRNA (adenine(1779)-N(6)/adenine(1780)-N(6))-dimethyltransferase activity [GO:0052909] (molecular function) Relationships: is a type of rRNA (adenine-N6,N6-)-dimethyltransferase activity [GO:0000179] Sources: RHEA:42780 Also known as: M(6)(2)A dimethylase activity Definition: Catalysis of the reaction: 4 S-adenosyl-L-methionine + adenine(1779)/adenine(1780) in 18S rRNA = 4 S-adenosyl-L-homocysteine + N(6)-dimethyladenine(1779)/N(6)-dimethyladenine(1780) in 18S rRNA.